{
  "term_id": "GO:0005634",
  "gene": "UniProtKB:O95067",
  "term_label": "nucleus",
  "gene_symbol": "CCNB2",
  "gene_name": "G2_mitotic-specific cyclin-B2"
}